positive regulation of neurofibrillary tangle assembly [GO:1902998] (biological process) Relationships: is a type of positive regulation of inclusion body assembly [GO:0090261]; is a type of regulation of neurofibrillary tangle assembly [GO:1902996]; positively regulates GO:1902988 Also known as: positive regulation of neurofibrillary tangle formation, up regulation of neurofibrillary tangle assembly, up regulation of neurofibrillary tangle formation, up-regulation of neurofibrillary tangle assembly, up-regulation of neurofibrillary tangle formation, upregulation of neurofibrillary tangle assembly, upregulation of neurofibrillary tangle formation, activation of flame-shaped neurofibrillary tangle assembly, activation of flame-shaped neurofibrillary tangle formation, activation of neurofibrillary tangle assembly, activation of neurofibrillary tangle formation, activation of star-shaped neurofibrillary tangle assembly, activation of star-shaped neurofibrillary tangle formation, positive regulation of flame-shaped neurofibrillary tangle assembly, positive regulation of flame-shaped neurofibrillary tangle formation, positive regulation of star-shaped neurofibrillary tangle assembly, positive regulation of star-shaped neurofibrillary tangle formation, up regulation of flame-shaped neurofibrillary tangle assembly, up regulation of flame-shaped neurofibrillary tangle formation, up regulation of star-shaped neurofibrillary tangle assembly, up regulation of star-shaped neurofibrillary tangle formation, up-regulation of flame-shaped neurofibrillary tangle assembly, up-regulation of flame-shaped neurofibrillary tangle formation, up-regulation of star-shaped neurofibrillary tangle assembly, up-regulation of star-shaped neurofibrillary tangle formation, upregulation of flame-shaped neurofibrillary tangle assembly, upregulation of flame-shaped neurofibrillary tangle formation, upregulation of star-shaped neurofibrillary tangle assembly, upregulation of star-shaped neurofibrillary tangle formation References: PMID:15897157 Sources: GOC:TermGenie, GOC:sjp, GO_REF:0000058 Definition: Any process that activates or increases the frequency, rate or extent of neurofibrillary tangle assembly.